{
  "term_label": "immune response-inhibiting cell surface receptor signaling pathway",
  "term_id": "GO:0002767",
  "gene_name": "Leukocyte immunoglobulin-like receptor subfamily B member 4",
  "gene": "UniProtKB:Q8NHJ6",
  "gene_symbol": "LILRB4"
}